{
  "gene": "UniProtKB:Q00526",
  "term_label": "cyclin-dependent protein kinase holoenzyme complex",
  "term_id": "GO:0000307",
  "gene_symbol": "CDK3",
  "gene_name": "Cyclin-dependent kinase 3"
}